D-xylose transmembrane transport [GO:0015753] (biological process) Relationships: is a type of pentose transmembrane transport [GO:0015750] Also known as: D-xylose transport Definition: The process in which D-xylose is transported across a lipid bilayer, from one side of a membrane to the other. D-xylose (the naturally occurring enantiomer is always D-) is a constituent of plant polysaccharides. Sources: GOC:ai